COPII-coated vesicle budding [GO:0090114] (BP) Sources: GOC:ascb_2009, GOC:dph, GOC:tb Relationships: is a type of vesicle budding from membrane [GO:0006900]; is part of endoplasmic reticulum to Golgi vesicle-mediated transport [GO:0006888] Definition: The evagination of an endoplasmic reticulum membrane, resulting in formation of a COPII-coated vesicle. Also known as: ER vesicle budding, ER exit, COPII vesicle budding